{
  "term_id": "GO:0017158",
  "term_label": "regulation of calcium ion-dependent exocytosis",
  "gene_name": "Synaptotagmin-7",
  "gene_symbol": "SYT7",
  "gene": "UniProtKB:O43581"
}